{
  "gene_name": "Transcription factor SOX-30",
  "gene_symbol": "SOX30",
  "term_id": "GO:1990837",
  "term_label": "sequence-specific double-stranded DNA binding",
  "gene": "UniProtKB:O94993"
}